{
  "gene_symbol": "RPIA",
  "gene_name": "Ribose-5-phosphate isomerase",
  "term_id": "GO:0009052",
  "gene": "UniProtKB:P49247",
  "term_label": "pentose-phosphate shunt, non-oxidative branch"
}